adhesion of symbiont infection cushion to host [GO:0075069] (BP) Sources: GOC:pamgo_curators Relationships: is a type of adhesion of symbiont infection structure to host [GO:0075001] Note: Note that this term should not be used to annotate gene products of the host. It should only be used to annotate those gene products from the symbiont involved in this process. Also known as: adhesion of symbiont infection cushion to host during symbiotic interaction Definition: The attachment of an infection cushion of the symbiont to its host via adhesion molecules. The host is defined as the larger of the organisms involved in a symbiotic interaction.